chitosanase activity [GO:0016977] (molecular function) Also known as: chitosan N-acetylglucosaminohydrolase activity Definition: Catalysis of the endohydrolysis of beta-1,4-linkages between N-acetyl-D-glucosamine and D-glucosamine residues in a partly acetylated chitosan. Sources: EC:3.2.1.132 Relationships: is_a hydrolase activity, hydrolyzing O-glycosyl compounds [GO:0004553]